response to capsazepine [GO:1901594] (biological process) Definition: Any process that results in a change in state or activity of a cell or an organism (in terms of movement, secretion, enzyme production, gene expression, etc.) as a result of a capsazepine stimulus. Subtypes: cellular response to capsazepine [GO:0072761] Sources: GOC:TermGenie Relationships: is_a response to nitrogen compound [GO:1901698]; is_a GO:1901700